insect pharynx development [GO:0160095] (BP) Definition: The process whose specific outcome is the progression of insect pharynx over time, from its formation to the mature structure. Relationships: is a type of pharynx development [GO:0060465] References: PMID:10952900